{
  "gene": "UniProtKB:Q86XS5",
  "term_id": "GO:0005615",
  "gene_symbol": "ANGPTL5",
  "term_label": "extracellular space",
  "gene_name": "Angiopoietin-related protein 5"
}